glucuronate transmembrane transport [GO:0015738] (biological process) Sources: GOC:krc Also known as: glucuronate transport Subtypes: D-glucuronate transmembrane transport [GO:0042874] Relationships: is a type of GO:0015736 Definition: The process in which glucuronate is transported across a lipid bilayer, from one side of a membrane to the other.